{
  "term_id": "GO:0005886",
  "term_label": "plasma membrane",
  "gene": "UniProtKB:Q9HCX4",
  "gene_name": "Short transient receptor potential channel 7",
  "gene_symbol": "TRPC7"
}